{
  "term_label": "mitochondrion",
  "term_id": "GO:0005739",
  "gene_name": "Aminomethyltransferase, mitochondrial",
  "gene_symbol": "AMT",
  "gene": "UniProtKB:P48728"
}